xylulose biosynthetic process [GO:0005999] (biological process) Sources: ISBN:0198547684 Relationships: is_a xylulose metabolic process [GO:0005997]; is a type of pentose biosynthetic process [GO:0019322] Definition: The chemical reactions and pathways resulting in the formation of xylulose, the ketopentose threo-2-pentulose. Also known as: xylulose anabolism, xylulose biosynthesis, xylulose formation, xylulose synthesis